{
  "gene": "UniProtKB:Q6ZT89",
  "gene_symbol": "SLC25A48",
  "term_label": "transmembrane transporter activity",
  "term_id": "GO:0022857",
  "gene_name": "Solute carrier family 25 member 48"
}